{
  "term_label": "Unknown cellular component",
  "term_id": "UNKNOWN:0003",
  "gene_symbol": "C2CD4C",
  "gene_name": "C2 calcium-dependent domain-containing protein 4C",
  "gene": "UniProtKB:Q8TF44"
}